N-isopropylammelide isopropylaminohydrolase activity [GO:0018764] (molecular function) Also known as: AtzC Sources: EC:3.5.4.42 Definition: Catalysis of the reaction: N-isopropylammelide + H2O = cyanuric acid + isopropylamine. Relationships: is a type of hydrolase activity, acting on carbon-nitrogen (but not peptide) bonds [GO:0016810]